mitochondrial tRNA wobble uridine modification [GO:0070899] (biological process) Relationships: is a type of tRNA wobble uridine modification [GO:0002098]; is a type of mitochondrial tRNA modification [GO:0070900] Sources: GOC:mah, GOC:mcc Definition: The process in which a uridine in position 34 of a mitochondrial tRNA is post-transcriptionally modified. Subtypes: GO:1990799